{
  "term_id": "GO:0005886",
  "gene_symbol": "CCKBR",
  "gene_name": "Gastrin_cholecystokinin type B receptor",
  "gene": "UniProtKB:P32239",
  "term_label": "plasma membrane"
}